{
  "gene_symbol": "INTS7",
  "term_id": "GO:0034472",
  "term_label": "snRNA 3'-end processing",
  "gene_name": "Integrator complex subunit 7",
  "gene": "UniProtKB:Q9NVH2"
}